{
  "term_id": "GO:0010960",
  "term_label": "magnesium ion homeostasis",
  "gene_symbol": "CNNM3",
  "gene": "UniProtKB:Q8NE01",
  "gene_name": "Metal transporter CNNM3"
}